plasma membrane proton-transporting V-type ATPase, V0 domain [GO:0000222] (cellular component) Sources: GOC:mah Definition: The V0 domain of a proton-transporting V-type ATPase found in the plasma membrane. Also known as: plasma membrane hydrogen ion-transporting ATPase V0 domain Relationships: is a type of proton-transporting V-type ATPase, V0 domain [GO:0033179]; is_a GO:0098797; is part of plasma membrane proton-transporting V-type ATPase complex [GO:0033181]